{
  "term_id": "GO:0097186",
  "gene_name": "Kallikrein-4",
  "term_label": "amelogenesis",
  "gene_symbol": "KLK4",
  "gene": "UniProtKB:Q9Y5K2"
}